{
  "term_id": "UNKNOWN:0003",
  "gene_name": "Putative uncharacterized protein encoded by LINC00173",
  "gene_symbol": "LINC00173",
  "term_label": "Unknown cellular component",
  "gene": "UniProtKB:Q6ZV60"
}